IgG immunoglobulin complex, circulating [GO:0071736] (cellular component) Also known as: IgG antibody, IgG1 antibody, IgG2 antibody, IgG2a antibody, IgG2b antibody, IgG2c antibody, IgG3 antibody, IgG4 antibody Note: Note that an IgG immunoglobulin complex has the function of antigen binding if a suitable antigen is available. Also, IgG isotypes vary by species. Sources: GOC:add, ISBN:0781765196 Definition: A protein complex composed of two identical immunoglobulin heavy chains of an IgG isotype and two identical immunoglobulin light chains, held together by disulfide bonds, and present in the extracellular space, in mucosal areas or other tissues, or circulating in the blood or lymph. Relationships: is a type of GO:0042571; is a type of IgG immunoglobulin complex [GO:0071735]